{
  "gene_name": "Heterogeneous nuclear ribonucleoprotein Q",
  "gene": "UniProtKB:O60506",
  "term_id": "GO:0070934",
  "gene_symbol": "SYNCRIP",
  "term_label": "CRD-mediated mRNA stabilization"
}